{
  "term_label": "Unknown molecular function",
  "term_id": "UNKNOWN:0001",
  "gene_name": "Putative uncharacterized protein encoded by LINC01387",
  "gene_symbol": "LINC01387",
  "gene": "UniProtKB:J3KSC0"
}